{
  "term_label": "response to starvation",
  "gene_name": "BCAS3 microtubule associated cell migration factor",
  "gene": "UniProtKB:Q9H6U6",
  "term_id": "GO:0042594",
  "gene_symbol": "BCAS3"
}